{
  "gene": "UniProtKB:Q8NAT2",
  "term_id": "UNKNOWN:0002",
  "gene_name": "Tudor domain-containing protein 5",
  "gene_symbol": "TDRD5",
  "term_label": "Unknown biological process"
}